interferon binding [GO:0019961] (molecular function) Also known as: IFN binding Subtypes: type I interferon binding [GO:0019962], type II interferon binding [GO:0019964], type III interferon binding [GO:0034347] References: PMID:9607096 Sources: Wikipedia:Interferon Relationships: is a type of cytokine binding [GO:0019955] Definition: Binding to an interferon, a protein produced by the immune systems of many animals in response to a challenge by a foreign agent.